{
  "gene_symbol": "PARP6",
  "gene": "UniProtKB:Q2NL67",
  "gene_name": "Protein mono-ADP-ribosyltransferase PARP6",
  "term_label": "kinase binding",
  "term_id": "GO:0019900"
}